{
  "gene_name": "Transmembrane protein 178B",
  "term_id": "UNKNOWN:0002",
  "gene_symbol": "TMEM178B",
  "term_label": "Unknown biological process",
  "gene": "UniProtKB:H3BS89"
}